{
  "gene_symbol": "HRC",
  "gene": "UniProtKB:P23327",
  "gene_name": "Sarcoplasmic reticulum histidine-rich calcium-binding protein",
  "term_label": "Unknown molecular function",
  "term_id": "UNKNOWN:0001"
}